{
  "gene": "UniProtKB:Q8IZV2",
  "term_id": "GO:0016020",
  "term_label": "membrane",
  "gene_symbol": "CMTM8",
  "gene_name": "CKLF-like MARVEL transmembrane domain-containing protein 8"
}